ruffle organization [GO:0031529] (biological process) Definition: A process that is carried out at the cellular level which results in the assembly, arrangement of constituent parts, or disassembly of a ruffle, a projection at the leading edge of a crawling cell. References: PMID:10036235 Sources: GOC:mah Subtypes: GO:0097178 Relationships: is_a plasma membrane bounded cell projection organization [GO:0120036] Also known as: ruffle organisation, ruffle organization and biogenesis